{
  "term_id": "GO:0017017",
  "gene_symbol": "DUSP10",
  "term_label": "MAP kinase tyrosine/serine/threonine phosphatase activity",
  "gene": "UniProtKB:Q9Y6W6",
  "gene_name": "Dual specificity protein phosphatase 10"
}